{
  "gene_name": "Protein transport protein Sec23A",
  "term_id": "GO:0090110",
  "term_label": "COPII-coated vesicle cargo loading",
  "gene_symbol": "SEC23A",
  "gene": "UniProtKB:Q15436"
}